{
  "gene": "UniProtKB:A2RUB1",
  "gene_symbol": "MEIOC",
  "gene_name": "Meiosis-specific coiled-coil domain-containing protein MEIOC",
  "term_label": "mRNA stabilization",
  "term_id": "GO:0048255"
}